{
  "term_label": "Unknown molecular function",
  "term_id": "UNKNOWN:0001",
  "gene_name": "KICSTOR complex protein ITFG2",
  "gene": "UniProtKB:Q969R8",
  "gene_symbol": "ITFG2"
}